{
  "gene_symbol": "HCST",
  "gene": "UniProtKB:Q9UBK5",
  "term_id": "GO:0005102",
  "term_label": "signaling receptor binding",
  "gene_name": "Hematopoietic cell signal transducer"
}